{
  "gene": "UniProtKB:Q13410",
  "gene_name": "Butyrophilin subfamily 1 member A1",
  "term_id": "GO:0009897",
  "term_label": "external side of plasma membrane",
  "gene_symbol": "BTN1A1"
}